regulation of fibroblast growth factor receptor signaling pathway [GO:0040036] (biological process) Definition: Any process that modulates the frequency, rate or extent of fibroblast growth factor receptor signaling pathway activity. Sources: GOC:go_curators Relationships: is a type of regulation of signal transduction [GO:0009966]; is a type of regulation of cellular response to growth factor stimulus [GO:0090287]; regulates fibroblast growth factor receptor signaling pathway [GO:0008543] Also known as: regulation of FGF receptor signaling pathway, regulation of FGF receptor signalling pathway, regulation of FGFR signaling pathway Subtypes: negative regulation of fibroblast growth factor receptor signaling pathway [GO:0040037], positive regulation of fibroblast growth factor receptor signaling pathway [GO:0045743], regulation of fibroblast growth factor receptor signaling pathway involved in neural plate anterior/posterior pattern formation [GO:2000313], regulation of fibroblast growth factor receptor signaling pathway involved in ureteric bud formation [GO:2000702]